{
  "gene": "UniProtKB:Q8IWT1",
  "gene_symbol": "SCN4B",
  "gene_name": "Sodium channel subunit beta-4",
  "term_label": "regulation of ventricular cardiac muscle cell membrane repolarization",
  "term_id": "GO:0060307"
}